{
  "gene_name": "YEATS domain-containing protein 2",
  "term_id": "GO:0140672",
  "term_label": "ATAC complex",
  "gene_symbol": "YEATS2",
  "gene": "UniProtKB:Q9ULM3"
}